{
  "gene_name": "Tyrosine-protein kinase RYK",
  "term_label": "receptor complex",
  "term_id": "GO:0043235",
  "gene": "UniProtKB:P34925",
  "gene_symbol": "RYK"
}